{
  "gene_name": "Calcium-binding tyrosine phosphorylation-regulated protein",
  "term_id": "GO:0005509",
  "term_label": "calcium ion binding",
  "gene_symbol": "CABYR",
  "gene": "UniProtKB:O75952"
}